{
  "term_label": "Unknown molecular function",
  "term_id": "UNKNOWN:0001",
  "gene_name": "Putative F-box_LRR-repeat protein 21",
  "gene": "UniProtKB:Q9UKT6",
  "gene_symbol": "FBXL21P"
}